{
  "term_label": "transmembrane transporter activity",
  "gene": "UniProtKB:O00624",
  "gene_symbol": "SLC17A2",
  "term_id": "GO:0022857",
  "gene_name": "Sodium-dependent phosphate transport protein 3"
}